{
  "gene_name": "Cannabinoid receptor 1",
  "term_id": "GO:0004930",
  "gene_symbol": "CNR1",
  "term_label": "G protein-coupled receptor activity",
  "gene": "UniProtKB:P21554"
}